plasmodesmatal cytoplasmic sleeve [GO:0009546] (cellular component) Definition: The space between the plasma membrane and the desmotubule of a plasmodesma. References: PMID:29880547 Also known as: plasmodesmatal cytoplasmic annulus Relationships: is a type of cellular anatomical structure [GO:0110165]; BFO_0000050 GO:0005886; is part of plasmodesma [GO:0009506]